{
  "term_id": "GO:0007169",
  "gene": "UniProtKB:P08922",
  "gene_name": "Proto-oncogene tyrosine-protein kinase ROS",
  "gene_symbol": "ROS1",
  "term_label": "cell surface receptor protein tyrosine kinase signaling pathway"
}